G2/M transition of mitotic cell cycle [GO:0000086] (biological process) Relationships: is a type of GO:0044772; is a type of GO:0044839 Regulation: regulated by GO:0010389; positively regulated by positive regulation of G2/M transition of mitotic cell cycle [GO:0010971]; negatively regulated by negative regulation of G2/M transition of mitotic cell cycle [GO:0010972] Definition: The mitotic cell cycle transition by which a cell in G2 commits to M phase. The process begins when the kinase activity of M cyclin/CDK complex reaches a threshold high enough for the cell cycle to proceed. This is accomplished by activating a positive feedback loop that results in the accumulation of unphosphorylated and active M cyclin/CDK complex. Also known as: mitotic G2/M transition Sources: GOC:mtg_cell_cycle